{
  "gene_name": "Large ribosomal subunit protein P2",
  "term_id": "UNKNOWN:0001",
  "term_label": "Unknown molecular function",
  "gene_symbol": "RPLP2",
  "gene": "UniProtKB:P05387"
}